{
  "gene_symbol": "STAT5B",
  "gene_name": "Signal transducer and activator of transcription 5B",
  "term_id": "GO:0000978",
  "gene": "UniProtKB:P51692",
  "term_label": "RNA polymerase II cis-regulatory region sequence-specific DNA binding"
}